{
  "term_label": "axon guidance",
  "gene_name": "Ephrin type-B receptor 3",
  "term_id": "GO:0007411",
  "gene": "UniProtKB:P54753",
  "gene_symbol": "EPHB3"
}